negative regulation of mating-type specific transcription, DNA-templated [GO:0045894] (biological process) Definition: Any mating-type specific process that stops, prevents or reduces the rate of cellular DNA-templated transcription. Relationships: is a type of regulation of mating-type specific transcription, DNA-templated [GO:0007532]; is a type of negative regulation of DNA-templated transcription [GO:0045892] Also known as: down regulation of transcription, mating-type specific, down-regulation of transcription, mating-type specific, downregulation of transcription, mating-type specific, negative regulation of mating-type specific transcription, DNA-dependent, inhibition of transcription, mating-type specific Sources: GOC:go_curators, GOC:txnOH